regulation of superoxide anion generation [GO:0032928] (biological process) Sources: GOC:mah Subtypes: negative regulation of superoxide anion generation [GO:0032929], GO:0032930 Also known as: regulation of superoxide release Definition: Any process that modulates the frequency, rate or extent of enzymatic generation of superoxide by a cell. Relationships: is a type of regulation of superoxide metabolic process [GO:0090322]; regulates superoxide anion generation [GO:0042554]